{
  "gene_name": "Homeobox protein Hox-A2",
  "gene_symbol": "HOXA2",
  "term_label": "DNA-binding transcription factor activity, RNA polymerase II-specific",
  "gene": "UniProtKB:O43364",
  "term_id": "GO:0000981"
}